{
  "gene": "UniProtKB:Q12766",
  "gene_name": "HMG domain-containing protein 3",
  "gene_symbol": "HMGXB3",
  "term_id": "UNKNOWN:0003",
  "term_label": "Unknown cellular component"
}